response to magnesium ion [GO:0032026] (biological process) Sources: GOC:mah Relationships: is a type of response to metal ion [GO:0010038] Subtypes: GO:0071286 Definition: Any process that results in a change in state or activity of a cell or an organism (in terms of movement, secretion, enzyme production, gene expression, etc.) as a result of a magnesium ion stimulus.